siRNA catabolic process [GO:0140746] (biological process) Definition: The chemical reactions and pathways resulting in the breakdown of small interfering RNA transcripts (siRNAs). Relationships: is a type of RNA catabolic process [GO:0006401] References: PMID:25928405